metamorphosis [GO:0007552] (biological process) Definition: A biological process in which an animal physically develops after birth or hatching, involving a conspicuous and relatively abrupt change in the animal's form or structure. Examples include the change from tadpole to frog, and the change from larva to adult. An example of this is found in Drosophila melanogaster. Relationships: is a type of multicellular organism development [GO:0007275] Sources: GOC:sensu, ISBN:0198506732, ISBN:0721662544